{
  "term_id": "UNKNOWN:0001",
  "gene_symbol": "TMEM235",
  "gene": "UniProtKB:A6NFC5",
  "gene_name": "Transmembrane protein 235",
  "term_label": "Unknown molecular function"
}